protein serine/threonine phosphatase complex [GO:0008287] (CC) Definition: A complex, normally consisting of a catalytic and a regulatory subunit, which catalyzes the removal of a phosphate group from a serine or threonine residue of a protein. Sources: GOC:bf Relationships: is a type of GO:1903293 Subtypes: protein phosphatase type 2A complex [GO:0000159], protein phosphatase type 1 complex [GO:0000164], GO:0005955, GO:0005963, GO:0017023, protein phosphatase 4 complex [GO:0030289], GO:0045253, Nem1-Spo7 phosphatase complex [GO:0071595], GO:1990567